{
  "gene_symbol": "CXCL12",
  "gene_name": "Stromal cell-derived factor 1",
  "term_id": "GO:0009897",
  "gene": "UniProtKB:P48061",
  "term_label": "external side of plasma membrane"
}